DNA (cytosine-5-)-methyltransferase activity [GO:0003886] (molecular function) Definition: Catalysis of the reaction: a 2'-deoxycytidine in DNA + S-adenosyl-L-methionine = a 5-methyl-2'-deoxycytidine in DNA + H+ + S-adenosyl-L-homocysteine. Sources: RHEA:13681 Also known as: DNA cytosine methylase activity, DNA-cytosine methyltransferase activity, cytosine DNA methylase activity, cytosine DNA methyltransferase activity, deoxyribonucleic methylase activity, site-specific DNA-methyltransferase (cytosine-specific) activity, DNA 5-cytosine methylase activity, DNA cytosine C(5) methylase activity, DNA cytosine C5 methylase activity, DNA-cytosine 5-methylase activity, S-adenosyl-L-methionine:DNA (cytosine-5-)-methyltransferase activity, cytosine 5-methyltransferase activity, cytosine-specific DNA methyltransferase activity, deoxyribonucleic (cytosine-5-)-methyltransferase activity, deoxyribonucleic acid (cytosine-5-)-methyltransferase activity, methylphosphotriester-DNA methyltransferase activity, modification methylase activity, restriction-modification system activity, type II DNA methylase activity Subtypes: DNA (cytosine-5-)-methyltransferase activity, acting on CpG substrates [GO:0051718], DNA (cytosine-5-)-methyltransferase activity, acting on CpN substrates [GO:0051719], DNA (cytosine-5-)-methyltransferase activity, acting on CpNpG substrates [GO:0051720], GO:0120328 Relationships: is a type of GO:0008757; is a type of GO:0009008